collagen metabolic process [GO:0032963] (biological process) Also known as: collagen metabolism Definition: The chemical reactions and pathways involving collagen, any of a group of fibrous proteins of very high tensile strength that form the main component of connective tissue in animals. Collagen is highly enriched in glycine (some regions are 33% glycine) and proline, occurring predominantly as 3-hydroxyproline (about 20%). Subtypes: collagen catabolic process [GO:0030574], GO:0032964 Regulation: regulated by regulation of collagen metabolic process [GO:0010712]; negatively regulated by negative regulation of collagen metabolic process [GO:0010713]; RO_0002213 by GO:0010714 Sources: GOC:mah, ISBN:0198506732 Relationships: is a type of metabolic process [GO:0008152]